chemorepulsion of branchiomotor neuron axon in branchial arch mesenchyme [GO:0021790] (biological process) Relationships: is a type of branchiomotor neuron axon guidance in branchial arch mesenchyme [GO:0021789]; is_a chemorepulsion of branchiomotor axon [GO:0021793] Also known as: negative chemotaxis of branchiomotor neuron axon in branchial arch mesenchyme References: PMID:14699587 Sources: GOC:cls, GOC:dgh, GOC:dph, GOC:jid, GO_REF:0000021 Definition: The process in which a branchiomotor neuron growth cone in the branchial arch mesenchyme is directed to a specific target site in the branchial arch mesenchyme in response to a repulsive chemical cue. Branchiomotor neurons are located in the hindbrain and innervate branchial arch-derived muscles that control jaw movements, facial expression, the larynx, and the pharynx.